{
  "gene_name": "Keratin, type II cytoskeletal 2 oral",
  "gene": "UniProtKB:Q01546",
  "term_label": "keratin filament",
  "term_id": "GO:0045095",
  "gene_symbol": "KRT76"
}